{
  "term_id": "GO:0018149",
  "gene_symbol": "F13A1",
  "gene_name": "Coagulation factor XIII A chain",
  "gene": "UniProtKB:P00488",
  "term_label": "peptide cross-linking"
}